parturition [GO:0007567] (biological process) Also known as: giving birth, egg laying Sources: ISBN:0198506732 Relationships: is a type of multi-organism reproductive process [GO:0044703]; is a type of multi-multicellular organism process [GO:0044706] Definition: The reproductive process in which the parent is separated from its offspring either by giving birth to live young or by laying eggs.